{
  "gene_name": "4-hydroxyphenylpyruvate dioxygenase",
  "term_label": "4-hydroxyphenylpyruvate dioxygenase activity",
  "term_id": "GO:0003868",
  "gene": "UniProtKB:P32754",
  "gene_symbol": "HPD"
}